{
  "term_label": "adherens junction",
  "gene": "UniProtKB:Q9ULB4",
  "gene_name": "Cadherin-9",
  "gene_symbol": "CDH9",
  "term_id": "GO:0005912"
}